{
  "term_label": "double-strand break repair",
  "gene": "UniProtKB:Q8IYW5",
  "gene_name": "E3 ubiquitin-protein ligase RNF168",
  "gene_symbol": "RNF168",
  "term_id": "GO:0006302"
}